PAT complex [GO:0160005] (cellular component) Relationships: is a type of GO:0098796; is a type of GO:0140534; is part of endoplasmic reticulum membrane [GO:0005789] Note: PAT complex functions by shielding exposed hydrophilicity of transmembrane domains (TMDs) to prevent premature degradation and promote proper folding and bundling of TMDs. Definition: A transmembrane protein complex located in the endoplasmic reticulum (ER) involved in the correct folding of multipass membrane proteins in the ER membrane. In human, the substrate-binding Asterix (PAT10, WDR83OS) forms an obligate heterodimer with CCDC47. References: PMID:32814900, PMID:33082068, PMID:33960686